{
  "gene": "UniProtKB:Q8N5Y8",
  "term_label": "endoplasmic reticulum unfolded protein response",
  "gene_name": "Protein mono-ADP-ribosyltransferase PARP16",
  "gene_symbol": "PARP16",
  "term_id": "GO:0030968"
}